pyrimidine ribonucleoside diphosphate catabolic process [GO:0009195] (biological process) Subtypes: TDP catabolic process [GO:0006245], UDP catabolic process [GO:0006256], GO:0046706 Sources: GOC:go_curators, ISBN:0198506732 Relationships: is a type of pyrimidine nucleoside diphosphate catabolic process [GO:0009140]; is a type of GO:0009191; is a type of pyrimidine ribonucleoside diphosphate metabolic process [GO:0009193] Definition: The chemical reactions and pathways resulting in the breakdown of pyrimidine ribonucleoside diphosphate, a compound consisting of a pyrimidine base linked to a ribose sugar esterified with diphosphate on the sugar. Also known as: pyrimidine ribonucleoside diphosphate breakdown, pyrimidine ribonucleoside diphosphate catabolism, pyrimidine ribonucleoside diphosphate degradation